{
  "gene": "UniProtKB:Q9C0B0",
  "term_label": "Unknown cellular component",
  "gene_name": "RING finger protein unkempt homolog",
  "term_id": "UNKNOWN:0003",
  "gene_symbol": "UNK"
}